{
  "term_id": "GO:0000149",
  "term_label": "SNARE binding",
  "gene_name": "Syntaxin-12",
  "gene_symbol": "STX12",
  "gene": "UniProtKB:Q86Y82"
}